{
  "gene_symbol": "UBE2T",
  "term_id": "GO:0061631",
  "gene_name": "Ubiquitin-conjugating enzyme E2 T",
  "term_label": "ubiquitin conjugating enzyme activity",
  "gene": "UniProtKB:Q9NPD8"
}